1-phenylethanol dehydrogenase activity [GO:0018449] (molecular function) Definition: Catalysis of the reaction: (S)-1-phenylethanol + NAD+ = acetophenone + H+ + NADH. Sources: RHEA:28198 Relationships: is a type of oxidoreductase activity, acting on CH-OH group of donors [GO:0016614]